{
  "term_id": "GO:0019843",
  "gene": "UniProtKB:Q68CQ4",
  "gene_name": "U3 small nucleolar RNA-associated protein 25 homolog",
  "term_label": "rRNA binding",
  "gene_symbol": "UTP25"
}